{
  "term_id": "GO:0005739",
  "gene": "UniProtKB:Q14409",
  "gene_name": "Glycerol kinase 3",
  "gene_symbol": "GK3",
  "term_label": "mitochondrion"
}